{
  "term_label": "plasma membrane",
  "gene_symbol": "PTK6",
  "gene_name": "Protein-tyrosine kinase 6",
  "gene": "UniProtKB:Q13882",
  "term_id": "GO:0005886"
}